regulation of anatomical structure morphogenesis [GO:0022603] (biological process) Relationships: is_a regulation of developmental process [GO:0050793]; regulates anatomical structure morphogenesis [GO:0009653] Also known as: regulation of morphogenesis Definition: Any process that modulates the frequency, rate or extent of anatomical structure morphogenesis. Subtypes: GO:0002085, regulation of germinal center formation [GO:0002634], regulation of gastrulation [GO:0010470], regulation of mitochondrial fusion [GO:0010635], regulation of somitogenesis [GO:0014807], regulation of cell morphogenesis [GO:0022604], regulation of angioblast cell migration involved in selective angioblast sprouting [GO:0035477], regulation of angiogenesis [GO:0045765], regulation of sprouting of injured axon [GO:0048686], regulation of dendrite morphogenesis [GO:0048814], regulation of axonogenesis [GO:0050770], GO:0060312, positive regulation of mammary placode formation by mesenchymal-epithelial signaling [GO:0060617], GO:0060688, GO:0060808, GO:0061001, regulation of hair follicle placode formation [GO:0061168], regulation of appressorium formation [GO:0075017], regulation of formation by symbiont of haustorium for nutrient acquisition from host [GO:0075045], GO:0075188, regulation of penetration hypha formation [GO:0075202], GO:0075329, GO:0090140, regulation of neural crest formation [GO:0090299], regulation of nematode male tail tip morphogenesis [GO:0110037], regulation of imaginal disc-derived leg joint morphogenesis [GO:0110137], regulation of shoot system morphogenesis [GO:1900618], GO:1901490, GO:1905140, regulation of morphogenesis of an epithelium [GO:1905330], regulation of plant organ morphogenesis [GO:1905421], regulation of plant organ formation [GO:1905428], regulation of artery morphogenesis [GO:1905651], regulation of animal organ morphogenesis [GO:2000027], negative regulation of blood vessel morphogenesis [GO:2000181], regulation of optic nerve formation [GO:2000595] Sources: GOC:mah